{
  "gene_name": "Small ribosomal subunit protein uS12",
  "gene_symbol": "RPS23",
  "term_id": "GO:0022627",
  "term_label": "cytosolic small ribosomal subunit",
  "gene": "UniProtKB:P62266"
}